vasoconstriction by vasopressin involved in systemic arterial blood pressure control [GO:0002006] (biological process) Also known as: vasopressin mediated vasoconstriction involved in systemic arterial blood pressure control Definition: The decrease in blood vessel diameter as a result of the release of vasopressin into the blood stream. Sources: GOC:dph, GOC:mtg_cardio, GOC:tb, ISBN:0721643949 Relationships: is a type of positive regulation of systemic arterial blood pressure [GO:0003084]; is a type of vasoconstriction [GO:0042310]; is part of regulation of systemic arterial blood pressure by vasopressin [GO:0001992]